{
  "term_id": "GO:0005634",
  "term_label": "nucleus",
  "gene_symbol": "CCNK",
  "gene": "UniProtKB:O75909",
  "gene_name": "Cyclin-K"
}